{
  "gene_name": "Protein S100-A8",
  "gene_symbol": "S100A8",
  "gene": "UniProtKB:P05109",
  "term_label": "calcium ion binding",
  "term_id": "GO:0005509"
}